{
  "gene_name": "SH2 domain-containing protein 2A",
  "gene": "UniProtKB:Q9NP31",
  "term_id": "GO:0042110",
  "gene_symbol": "SH2D2A",
  "term_label": "T cell activation"
}